{
  "gene_name": "Spindle and kinetochore-associated protein 1",
  "term_id": "GO:0000940",
  "term_label": "outer kinetochore",
  "gene_symbol": "SKA1",
  "gene": "UniProtKB:Q96BD8"
}